{
  "term_id": "GO:0005615",
  "gene_symbol": "IFNA14",
  "gene": "UniProtKB:P01570",
  "gene_name": "Interferon alpha-14",
  "term_label": "extracellular space"
}